{
  "term_label": "immune response-inhibiting cell surface receptor signaling pathway",
  "gene_symbol": "A0A1W2PRS3",
  "term_id": "GO:0002767",
  "gene_name": "Immunoglobulin subtype domain-containing protein",
  "gene": "UniProtKB:A0A1W2PRS3"
}